{
  "term_label": "regulation of synaptic transmission, glutamatergic",
  "gene_symbol": "GRM3",
  "term_id": "GO:0051966",
  "gene_name": "Metabotropic glutamate receptor 3",
  "gene": "UniProtKB:Q14832"
}